trans-aconitate 2-methyltransferase activity [GO:0030798] (molecular function) Also known as: S-adenosyl-L-methionine:(E)-prop-1-ene-1,2,3-tricarboxylate 2'-O-methyltransferase activity Definition: Catalysis of the reaction: S-adenosyl-L-methionine + trans-aconitate = (E)-3-(methoxycarbonyl)pent-2-enedioate + S-adenosyl-L-homocysteine. Relationships: is a type of S-adenosylmethionine-dependent methyltransferase activity [GO:0008757] Sources: EC:2.1.1.144, RHEA:14969